trans-cinnamate-CoA ligase activity [GO:0106290] (molecular function) References: PMID:22649270 Sources: RHEA:64788 Relationships: is a type of CoA-ligase activity [GO:0016405] Definition: Catalysis of the reaction: (E)-cinnamate + ATP + CoA = (E)-cinnamoyl-CoA + AMP + diphosphate.